{
  "gene_symbol": "EXOSC3",
  "term_id": "GO:0071051",
  "gene": "UniProtKB:Q9NQT5",
  "gene_name": "Exosome complex component RRP40",
  "term_label": "poly(A)-dependent snoRNA 3'-end processing"
}